ciliary cap [GO:0061822] (cellular component) Relationships: is a type of cellular anatomical structure [GO:0110165]; is part of cilium [GO:0005929] Definition: An intracellular compartmentalized cilium structure found in insect spermatids which is bounded by a membrane derived from the invagination of the cell membrane that remains associated with the primary cilium as it is internalized. The ciliary cap is maintained at the end of the axoneme distal to the centriole and is separated from the cytosolic axoneme/cytoplasm by a putative transition zone, which may extend into the ciliary cap, and include a structure at the base of the ciliary cap termed the ring centriole. References: PMID:25447994, PMID:27646273 Also known as: spermatid ciliary cap